{
  "gene_name": "NADPH oxidase 3",
  "gene": "UniProtKB:Q9HBY0",
  "term_id": "GO:0043020",
  "gene_symbol": "NOX3",
  "term_label": "NADPH oxidase complex"
}